galactonate dehydratase activity [GO:0008869] (molecular function) Sources: EC:4.2.1.6, RHEA:18649 Relationships: is a type of GO:0016836 Also known as: D-galactonate dehydrase activity, D-galactonate dehydratase activity, D-galactonate hydro-lyase (2-dehydro-3-deoxy-D-galactonate-forming), D-galactonate hydro-lyase activity Definition: Catalysis of the reaction: D-galactonate = 2-dehydro-3-deoxy-D-galactonate + H2O.